{
  "gene_name": "C-C motif chemokine 22",
  "term_label": "chemokine-mediated signaling pathway",
  "term_id": "GO:0070098",
  "gene": "UniProtKB:O00626",
  "gene_symbol": "CCL22"
}